regulation of establishment of protein-containing complex localization to telomere [GO:1904913] (biological process) Definition: Any process that modulates the frequency, rate or extent of establishment of the localization of a protein-containing macromolecular complex to a telomere. References: PMID:26586433 Sources: GOC:BHF, GOC:BHF_telomere, GOC:TermGenie, GOC:rph, GO_REF:0000058 Subtypes: GO:1904914, GO:1904915 Also known as: regulation of establishment of macromolecular complex localisation to telomere, regulation of establishment of macromolecular complex localization to telomere Relationships: is a type of regulation of localization [GO:0032879]; RO_0002211 establishment of protein-containing complex localization to telomere [GO:0097695]